{
  "gene_symbol": "SLC8A3",
  "gene_name": "Sodium_calcium exchanger 3",
  "gene": "UniProtKB:P57103",
  "term_id": "GO:0030424",
  "term_label": "axon"
}